{
  "gene_name": "Akirin-1",
  "gene_symbol": "AKIRIN1",
  "term_label": "positive regulation of transcription by RNA polymerase II",
  "gene": "UniProtKB:Q9H9L7",
  "term_id": "GO:0045944"
}